{
  "gene": "UniProtKB:Q9GZN0",
  "term_id": "GO:0007186",
  "gene_name": "Probable G-protein coupled receptor 88",
  "gene_symbol": "GPR88",
  "term_label": "G protein-coupled receptor signaling pathway"
}